{
  "gene": "UniProtKB:P48509",
  "gene_name": "CD151 antigen",
  "term_id": "UNKNOWN:0001",
  "term_label": "Unknown molecular function",
  "gene_symbol": "CD151"
}